{
  "gene": "UniProtKB:Q14154",
  "term_id": "GO:0140468",
  "term_label": "HRI-mediated signaling",
  "gene_symbol": "DELE1",
  "gene_name": "DAP3-binding cell death enhancer 1"
}